9,10-dihydroxystearate hydroxylase activity [GO:0103006] (molecular function) Relationships: is a type of GO:0016709 Definition: Catalysis of the reaction: H+ + (9R,10S)-dihydroxystearate + O2 + NADPH = 9,10,18-trihydroxystearate + H2O + NADP. Sources: GOC:pz